{
  "gene_name": "Transcription intermediary factor 1-beta",
  "term_label": "innate immune response",
  "gene": "UniProtKB:Q13263",
  "gene_symbol": "TRIM28",
  "term_id": "GO:0045087"
}